negative regulation of antibacterial peptide biosynthetic process [GO:0002809] (biological process) Subtypes: negative regulation of biosynthetic process of antibacterial peptides active against Gram-negative bacteria [GO:0002814], negative regulation of biosynthetic process of antibacterial peptides active against Gram-positive bacteria [GO:0002817] Sources: GOC:add Relationships: is a type of negative regulation of antibacterial peptide production [GO:0002787]; is_a negative regulation of antimicrobial peptide biosynthetic process [GO:0002806]; is a type of regulation of antibacterial peptide biosynthetic process [GO:0002808]; negatively regulates GO:0002780 Definition: Any process that stops, prevents, or reduces the frequency, rate, or extent of antibacterial peptide biosynthesis. Also known as: down regulation of antibacterial peptide biosynthetic process, down-regulation of antibacterial peptide biosynthetic process, downregulation of antibacterial peptide biosynthetic process, inhibition of antibacterial peptide biosynthetic process